{
  "term_id": "UNKNOWN:0001",
  "gene_name": "Proteasome inhibitor PI31 subunit",
  "gene": "UniProtKB:Q92530",
  "term_label": "Unknown molecular function",
  "gene_symbol": "PSMF1"
}